{
  "gene": "UniProtKB:Q96RD1",
  "gene_symbol": "OR6C1",
  "gene_name": "Olfactory receptor 6C1",
  "term_label": "plasma membrane",
  "term_id": "GO:0005886"
}